manganese ion export across plasma membrane [GO:0140048] (BP) References: PMID:25319704 Definition: The directed movement of manganese ions from inside of a cell, across the plasma membrane and into the extracellular region. Also known as: manganese ion export from cell Relationships: is a type of manganese ion transmembrane transport [GO:0071421]; is a type of export across plasma membrane [GO:0140115]